dormancy exit of symbiont in host [GO:0085016] (biological process) Relationships: is a type of dormancy process [GO:0022611]; is a type of GO:0044114 Also known as: resuscitation of symbiont Definition: Exit from dormant state, also known as resuscitation, of the symbiont within the host organism. Sources: GOC:jl